{
  "term_id": "GO:0030971",
  "gene_symbol": "SHC2",
  "term_label": "receptor tyrosine kinase binding",
  "gene_name": "SHC-transforming protein 2",
  "gene": "UniProtKB:P98077"
}